{
  "term_id": "GO:0120212",
  "gene_symbol": "SPATC1L",
  "gene_name": "Speriolin-like protein",
  "term_label": "sperm head-tail coupling apparatus",
  "gene": "UniProtKB:Q9H0A9"
}